negative regulation of synaptic vesicle exocytosis [GO:2000301] (biological process) Relationships: is a type of negative regulation of regulated secretory pathway [GO:1903306]; is a type of regulation of synaptic vesicle exocytosis [GO:2000300]; negatively regulates synaptic vesicle exocytosis [GO:0016079] Subtypes: negative regulation of synaptic vesicle priming [GO:0010809], GO:0031631, negative regulation of calcium ion-dependent exocytosis of neurotransmitter [GO:1903234] Definition: Any process that stops, prevents or reduces the frequency, rate or extent of synaptic vesicle exocytosis. Sources: GOC:obol